{
  "gene": "UniProtKB:O60763",
  "term_id": "GO:0045056",
  "gene_name": "General vesicular transport factor p115",
  "gene_symbol": "USO1",
  "term_label": "transcytosis"
}